{
  "gene": "UniProtKB:Q96T37",
  "gene_name": "RNA-binding protein 15",
  "gene_symbol": "RBM15",
  "term_label": "regulation of alternative mRNA splicing, via spliceosome",
  "term_id": "GO:0000381"
}